{
  "gene_name": "X antigen family member 2",
  "term_label": "Unknown biological process",
  "term_id": "UNKNOWN:0002",
  "gene_symbol": "XAGE2",
  "gene": "UniProtKB:Q96GT9"
}